phosphonate dehydrogenase activity [GO:0050609] (MF) Also known as: NAD-dependent phosphite dehydrogenas activity, NAD:phosphite oxidoreductase activity, phosphite dehydrogenase activity, phosphonate:NAD+ oxidoreductase activity Relationships: is a type of oxidoreductase activity, acting on phosphorus or arsenic in donors, with NAD(P)+ as acceptor [GO:0050499] Definition: Catalysis of the reaction: H2O + NAD+ + phosphonate = 2 H+ + NADH + phosphate. Sources: EC:1.20.1.1, RHEA:13173